{
  "gene": "UniProtKB:Q9P2E3",
  "gene_name": "NFX1-type zinc finger-containing protein 1",
  "gene_symbol": "ZNFX1",
  "term_id": "GO:0031380",
  "term_label": "nuclear RNA-directed RNA polymerase complex"
}